{
  "term_id": "GO:1990316",
  "gene": "UniProtKB:Q9BSB4",
  "term_label": "Atg1/ULK1 kinase complex",
  "gene_symbol": "ATG101",
  "gene_name": "Autophagy-related protein 101"
}